{
  "term_label": "proteasome-mediated ubiquitin-dependent protein catabolic process",
  "term_id": "GO:0043161",
  "gene_name": "Kelch-like protein 40",
  "gene": "UniProtKB:Q2TBA0",
  "gene_symbol": "KLHL40"
}